{
  "gene_symbol": "CELF2-AS1",
  "gene_name": "Putative uncharacterized protein CELF2-AS1",
  "gene": "UniProtKB:Q8N7Q2",
  "term_id": "UNKNOWN:0002",
  "term_label": "Unknown biological process"
}